{
  "gene_symbol": "TRAV18",
  "term_label": "immunoglobulin complex",
  "term_id": "GO:0019814",
  "gene": "UniProtKB:A0A075B6X5",
  "gene_name": "T cell receptor alpha variable 18"
}